{
  "term_id": "GO:0007399",
  "gene_name": "Pikachurin",
  "gene": "UniProtKB:Q63HQ2",
  "gene_symbol": "EGFLAM",
  "term_label": "nervous system development"
}